regulation of mitochondrial mRNA catabolic process [GO:1905637] (biological process) References: PMID:27122350 Sources: GOC:TermGenie, GO_REF:0000058 Relationships: is_a regulation of mitochondrial RNA catabolic process [GO:0000960]; is a type of regulation of mRNA catabolic process [GO:0061013]; RO_0002211 mitochondrial mRNA catabolic process [GO:0000958] Definition: Any process that modulates the frequency, rate or extent of mitochondrial mRNA catabolic process. Subtypes: negative regulation of mitochondrial mRNA catabolic process [GO:1905638], positive regulation of mitochondrial mRNA catabolic process [GO:1905639]